{
  "gene_symbol": "TRBJ1-1",
  "term_id": "UNKNOWN:0003",
  "gene_name": "T cell receptor beta joining 1-1",
  "term_label": "Unknown cellular component",
  "gene": "UniProtKB:A0A0J9YXA8"
}